{
  "gene": "UniProtKB:P07948",
  "gene_symbol": "LYN",
  "term_id": "GO:0031175",
  "gene_name": "Tyrosine-protein kinase Lyn",
  "term_label": "neuron projection development"
}